{
  "term_label": "cell adhesion molecule binding",
  "term_id": "GO:0050839",
  "gene_name": "Teneurin-1",
  "gene_symbol": "TENM1",
  "gene": "UniProtKB:Q9UKZ4"
}